{
  "term_id": "GO:0004035",
  "gene_symbol": "ALPG",
  "gene_name": "Alkaline phosphatase, germ cell type",
  "gene": "UniProtKB:P10696",
  "term_label": "alkaline phosphatase activity"
}